ethylene metabolic process [GO:0009692] (biological process) Subtypes: ethylene biosynthetic process [GO:0009693], GO:0042457 Relationships: is_a olefin metabolic process [GO:1900673] Definition: The chemical reactions and pathways involving ethylene (C2-H4, ethene), a simple hydrocarbon gas that can function in plants as a growth regulator. Sources: ISBN:0387969845 Also known as: ethene metabolic process, ethene metabolism, ethylene metabolism